positive regulation of transcription by glucose [GO:0046016] (biological process) Sources: GOC:go_curators Definition: Any process involving glucose that activates or increases the rate of transcription. Relationships: is a type of carbon catabolite activation of transcription [GO:0045991]; is a type of regulation of transcription by glucose [GO:0046015] Also known as: up regulation of transcription by glucose, up-regulation of transcription by glucose, upregulation of transcription by glucose, activation of transcription by glucose, stimulation of transcription by glucose Subtypes: positive regulation of transcription from RNA polymerase II promoter by glucose [GO:0000432]